{
  "term_label": "calcium import into the mitochondrion",
  "gene_symbol": "MICU1",
  "gene_name": "Calcium uptake protein 1, mitochondrial",
  "term_id": "GO:0036444",
  "gene": "UniProtKB:Q9BPX6"
}